{
  "gene_name": "DDB1- and CUL4-associated factor 8-like protein 1",
  "gene": "UniProtKB:A6NGE4",
  "gene_symbol": "DCAF8L1",
  "term_id": "UNKNOWN:0002",
  "term_label": "Unknown biological process"
}